{
  "gene_symbol": "THAP6",
  "gene_name": "THAP domain-containing protein 6",
  "term_label": "Unknown cellular component",
  "gene": "UniProtKB:Q8TBB0",
  "term_id": "UNKNOWN:0003"
}